positive regulation of myofibroblast cell apoptotic process [GO:1904522] (biological process) Definition: Any process that activates or increases the frequency, rate or extent of myofibroblast cell apoptotic process. Also known as: positive regulation of MFB apoptotic process, up regulation of MFB apoptotic process, up regulation of myofibroblast cell apoptotic process, up-regulation of MFB apoptotic process, up-regulation of myofibroblast cell apoptotic process, upregulation of MFB apoptotic process, upregulation of myofibroblast cell apoptotic process, activation of MFB apoptosis, activation of MFB apoptotic process, activation of myofibroblast cell apoptosis, activation of myofibroblast cell apoptotic process, positive regulation of MFB apoptosis, positive regulation of myofibroblast cell apoptosis, up regulation of MFB apoptosis, up regulation of myofibroblast cell apoptosis, up-regulation of MFB apoptosis, up-regulation of myofibroblast cell apoptosis, upregulation of MFB apoptosis, upregulation of myofibroblast cell apoptosis References: PMID:26119034 Sources: GOC:TermGenie, GO_REF:0000058 Relationships: is a type of positive regulation of apoptotic process [GO:0043065]; is a type of regulation of myofibroblast cell apoptotic process [GO:1904520]; positively regulates myofibroblast cell apoptotic process [GO:1904516]